intracellular amino acid homeostasis [GO:0080144] (biological process) References: PMID:19955263 Relationships: is a type of intracellular chemical homeostasis [GO:0055082] Subtypes: intracellular cysteine homeostasis [GO:0080145], intracellular aspartate homeostasis [GO:0090459], intracellular threonine homeostasis [GO:0090460], intracellular glutamate homeostasis [GO:0090461], intracellular ornithine homeostasis [GO:0090462], intracellular lysine homeostasis [GO:0090463], intracellular histidine homeostasis [GO:0090464], intracellular arginine homeostasis [GO:0090465] Also known as: amino acid homeostasis, cellular amino acid homeostasis Definition: A homeostatic process involved in the maintenance of a steady state level of amino acids within a cell.